{
  "gene_symbol": "KIR2DS1",
  "gene": "UniProtKB:Q14954",
  "gene_name": "Killer cell immunoglobulin-like receptor 2DS1",
  "term_id": "GO:0002767",
  "term_label": "immune response-inhibiting cell surface receptor signaling pathway"
}